{
  "gene_symbol": "CAMP",
  "term_label": "antimicrobial humoral immune response mediated by antimicrobial peptide",
  "gene_name": "Cathelicidin antimicrobial peptide",
  "term_id": "GO:0061844",
  "gene": "UniProtKB:P49913"
}